{
  "term_id": "UNKNOWN:0001",
  "gene": "UniProtKB:P0C0L5",
  "gene_name": "Complement C4-B",
  "term_label": "Unknown molecular function",
  "gene_symbol": "C4B_2"
}